{
  "gene": "UniProtKB:Q9BUN1",
  "gene_name": "Protein MENT",
  "gene_symbol": "MENT",
  "term_id": "UNKNOWN:0003",
  "term_label": "Unknown cellular component"
}